{
  "gene_name": "Tropomodulin-3",
  "term_label": "myofibril",
  "term_id": "GO:0030016",
  "gene": "UniProtKB:Q9NYL9",
  "gene_symbol": "TMOD3"
}